RNA 7-methylguanosine cap binding [GO:0000340] (molecular function) Sources: GOC:krc Also known as: RNA m7G cap binding Definition: Binding to a 7-methylguanosine group added cotranscriptionally to the 5' end of RNA molecules transcribed by polymerase II. Relationships: is a type of RNA cap binding [GO:0000339]